{
  "gene_name": "Protein FAM236C",
  "term_id": "UNKNOWN:0001",
  "gene_symbol": "FAM236C",
  "gene": "UniProtKB:P0DP71",
  "term_label": "Unknown molecular function"
}